{
  "term_id": "GO:0000407",
  "term_label": "phagophore assembly site",
  "gene": "UniProtKB:Q96BY7",
  "gene_name": "Autophagy-related protein 2 homolog B",
  "gene_symbol": "ATG2B"
}